ephrin receptor binding [GO:0046875] (molecular function) Definition: Binding to an ephrin receptor. Relationships: is a type of signaling receptor binding [GO:0005102] Sources: GOC:ai Also known as: Eph receptor binding, GPI-linked ephrin, ephrin, transmembrane ephrin